regulation of MAPK cascade [GO:0043408] (biological process) Also known as: regulation of MAP kinase cascade, regulation of MAP kinase kinase kinase cascade, regulation of MAPKKK cascade, regulation of mitogen activated protein kinase cascade, regulation of mitogen activated protein kinase kinase kinase cascade, regulation of mitogen-activated protein kinase cascade, regulation of mitogen-activated protein kinase kinase kinase cascade Definition: Any process that modulates the frequency, rate or extent of signal transduction mediated by the MAP kinase (MAPK) cascade. Relationships: is a type of regulation of intracellular signal transduction [GO:1902531]; regulates GO:0000165 Sources: GOC:go_curators Subtypes: regulation of stress-activated MAPK cascade [GO:0032872], negative regulation of MAPK cascade [GO:0043409], positive regulation of MAPK cascade [GO:0043410], GO:0046328, regulation of ERK1 and ERK2 cascade [GO:0070372], regulation of ERK5 cascade [GO:0070376], regulation of pheromone response MAPK cascade [GO:0180039], GO:1900744